positive regulation of glycolytic process [GO:0045821] (biological process) Definition: Any process that activates or increases the frequency, rate or extent of glycolysis. Sources: GOC:go_curators Also known as: up regulation of glycolysis, up-regulation of glycolysis, upregulation of glycolysis, activation of glycolysis, stimulation of glycolysis Relationships: is a type of GO:0006110; is a type of GO:0033123; is a type of positive regulation of carbohydrate metabolic process [GO:0045913]; is a type of positive regulation of ATP metabolic process [GO:1903580]; positively regulates glycolytic process [GO:0006096] Subtypes: positive regulation of glycolytic process through fructose-6-phosphate [GO:1904540]